{
  "gene": "UniProtKB:Q5H9R7",
  "gene_name": "Serine_threonine-protein phosphatase 6 regulatory subunit 3",
  "term_id": "GO:0009966",
  "gene_symbol": "PPP6R3",
  "term_label": "regulation of signal transduction"
}